primary dendrite [GO:0150001] (cellular component) Sources: GOC:aruk, GOC:bc Relationships: is a type of dendrite [GO:0030425] Definition: A dendrite emerging from the cell body (the soma) of a neuron.